{
  "gene_name": "Putative ribosomal protein uL13-like",
  "term_label": "Unknown molecular function",
  "gene": "UniProtKB:Q6NVV1",
  "term_id": "UNKNOWN:0001",
  "gene_symbol": "RPL13AP3"
}